alpha4-beta1 integrin-CD63 complex [GO:0070519] (cellular component) Also known as: ITGA4-ITGB1-CD63 complex Relationships: is a type of plasma membrane protein complex [GO:0098797] Definition: A protein complex that consists of an alpha4-beta1 integrin complex bound to membrane protein CD63, a member of the tetraspan family. References: PMID:8757325